{
  "term_id": "GO:0005634",
  "gene_symbol": "SIX1",
  "gene": "UniProtKB:Q15475",
  "gene_name": "Homeobox protein SIX1",
  "term_label": "nucleus"
}